{
  "term_id": "GO:0035804",
  "gene": "UniProtKB:Q12836",
  "term_label": "structural constituent of egg coat",
  "gene_symbol": "ZP4",
  "gene_name": "Zona pellucida sperm-binding protein 4"
}